7SK snRNP [GO:0120259] (cellular component) References: PMID:18249148, PMID:28431135 Relationships: is a type of small nuclear ribonucleoprotein complex [GO:0030532] Definition: A ribonucleoprotein complex that contains the 7SK snRNA. The 7SK snRNP plays a central role in RNA polymerase II elongation control by regulating the availability of active P-TEFb. Also known as: snRNP 7SK